{
  "term_id": "GO:0004465",
  "gene": "UniProtKB:P54315",
  "gene_name": "Inactive pancreatic lipase-related protein 1",
  "term_label": "lipoprotein lipase activity",
  "gene_symbol": "PNLIPRP1"
}